peptide serotonyltransferase activity [GO:0120294] (molecular function) Definition: Catalysis of the reaction: L-glutaminyl-[protein] + serotonin = 5-serotonyl-L-glutamyl-[protein] + NH4(+). References: PMID:14697203 Sources: GOC:sp Relationships: is a type of GO:0016410 Subtypes: GO:0120295